{
  "gene_name": "Solute carrier family 35 member E2B",
  "gene": "UniProtKB:P0CK96",
  "gene_symbol": "SLC35E2B",
  "term_label": "antiporter activity",
  "term_id": "GO:0015297"
}